planar cell polarity pathway involved in cardiac muscle cell fate commitment [GO:0061345] (biological process) Relationships: is a type of Wnt signaling pathway, planar cell polarity pathway [GO:0060071]; is a type of non-canonical Wnt signaling pathway involved in heart development [GO:0061341] Definition: The series of molecular signals initiated by binding of a Wnt protein to a frizzled family receptor on the surface of the target cell, followed by propagation of the signal via effectors other than beta-catenin and contributing to a cardioblast being committed to a cardiac muscle cell fate. References: PMID:16860783 Sources: GOC:dph, GOC:mtg_heart